cardiolipin hydrolase activity [GO:0035755] (molecular function) References: PMID:17028579, PMID:21397848 Sources: GOC:sp Definition: Catalysis of the hydrolysis of cardiolipin (1,3-bis(3-phosphatidyl)glycerol), releasing phosphatidic acid (PA). Relationships: is a type of phospholipase activity [GO:0004620]; is_a phosphoric diester hydrolase activity [GO:0008081]